{
  "gene_symbol": "PCP4",
  "term_label": "calmodulin binding",
  "gene_name": "Calmodulin regulator protein PCP4",
  "term_id": "GO:0005516",
  "gene": "UniProtKB:P48539"
}